{
  "term_id": "UNKNOWN:0002",
  "gene_symbol": "CSNKA2IP",
  "gene": "UniProtKB:A0A1B0GTH6",
  "term_label": "Unknown biological process",
  "gene_name": "Casein kinase II subunit alpha'-interacting protein"
}